{
  "gene_name": "FACT complex subunit SSRP1",
  "gene": "UniProtKB:Q08945",
  "term_label": "nucleosome binding",
  "gene_symbol": "SSRP1",
  "term_id": "GO:0031491"
}